{
  "gene": "UniProtKB:P41439",
  "term_id": "GO:0009897",
  "term_label": "external side of plasma membrane",
  "gene_symbol": "FOLR3",
  "gene_name": "Folate receptor gamma"
}